{
  "gene_name": "Metallothionein-4",
  "gene": "UniProtKB:P47944",
  "gene_symbol": "MT4",
  "term_id": "GO:0071276",
  "term_label": "cellular response to cadmium ion"
}